establishment of monopolar cell polarity [GO:0061162] (biological process) Definition: The specification and formation of monopolar intracellular organization or cell growth patterns. Monopolar cell organization is directional organization along an axis. Sources: GOC:dph, GOC:vw Relationships: is a type of establishment of cell polarity [GO:0030010]; is a type of establishment or maintenance of monopolar cell polarity [GO:0061339] Subtypes: establishment of proximal/distal cell polarity [GO:0022606], establishment of apical/basal cell polarity [GO:0035089], cell growth mode switching, bipolar to monopolar [GO:0051524]